{
  "term_id": "GO:0061844",
  "gene_symbol": "CX3CL1",
  "term_label": "antimicrobial humoral immune response mediated by antimicrobial peptide",
  "gene_name": "Fractalkine",
  "gene": "UniProtKB:P78423"
}